{
  "gene": "UniProtKB:Q99453",
  "gene_symbol": "PHOX2B",
  "term_label": "DNA-binding transcription factor activity, RNA polymerase II-specific",
  "gene_name": "Paired mesoderm homeobox protein 2B",
  "term_id": "GO:0000981"
}